{
  "term_label": "vesicle budding from membrane",
  "term_id": "GO:0006900",
  "gene": "UniProtKB:O60641",
  "gene_name": "Clathrin coat assembly protein AP180",
  "gene_symbol": "SNAP91"
}